{
  "gene_name": "Double-stranded RNA-binding protein Staufen homolog 1",
  "term_label": "germ cell development",
  "gene_symbol": "STAU1",
  "term_id": "GO:0007281",
  "gene": "UniProtKB:O95793"
}